{
  "term_label": "double-stranded RNA binding",
  "term_id": "GO:0003725",
  "gene": "UniProtKB:Q96C10",
  "gene_symbol": "DHX58",
  "gene_name": "ATP-dependent RNA helicase DHX58"
}